{
  "gene_name": "Dynein axonemal assembly factor 3",
  "term_id": "GO:0070286",
  "term_label": "axonemal dynein complex assembly",
  "gene_symbol": "DNAAF3",
  "gene": "UniProtKB:Q8N9W5"
}